{
  "gene": "UniProtKB:Q96HY7",
  "gene_name": "2-oxoadipate dehydrogenase complex component E1",
  "term_id": "UNKNOWN:0002",
  "term_label": "Unknown biological process",
  "gene_symbol": "DHTKD1"
}